regulation of smooth muscle tissue development [GO:1905899] (biological process) References: PMID:14709716 Sources: GOC:TermGenie, GOC:bhm, GO_REF:0000058 Definition: Any process that modulates the frequency, rate or extent of smooth muscle tissue development. Relationships: is a type of regulation of muscle tissue development [GO:1901861]; regulates GO:0048745 Subtypes: negative regulation of smooth muscle tissue development [GO:1905900], positive regulation of smooth muscle tissue development [GO:1905901]